{
  "gene_name": "Dihydropyrimidinase-related protein 2",
  "gene_symbol": "DPYSL2",
  "term_label": "Unknown biological process",
  "term_id": "UNKNOWN:0002",
  "gene": "UniProtKB:Q16555"
}